{
  "gene": "UniProtKB:Q8N1L9",
  "gene_name": "Basic leucine zipper transcriptional factor ATF-like 2",
  "term_label": "regulation of transcription by RNA polymerase II",
  "gene_symbol": "BATF2",
  "term_id": "GO:0006357"
}